{
  "term_label": "transforming growth factor beta binding",
  "term_id": "GO:0050431",
  "gene": "UniProtKB:Q86YC3",
  "gene_symbol": "NRROS",
  "gene_name": "Transforming growth factor beta activator LRRC33"
}